{
  "gene": "UniProtKB:Q16674",
  "term_id": "GO:0030198",
  "gene_name": "Melanoma-derived growth regulatory protein",
  "gene_symbol": "MIA",
  "term_label": "extracellular matrix organization"
}